positive regulation of carotenoid biosynthetic process [GO:1904143] (BP) Definition: Any process that activates or increases the frequency, rate or extent of carotenoid biosynthetic process. Also known as: positive regulation of carotenoid anabolism, positive regulation of carotenoid biosynthesis, positive regulation of carotenoid formation, positive regulation of carotenoid synthesis, up regulation of carotenoid anabolism, up regulation of carotenoid biosynthesis, up regulation of carotenoid biosynthetic process, up regulation of carotenoid formation, up regulation of carotenoid synthesis, up-regulation of carotenoid anabolism, up-regulation of carotenoid biosynthesis, up-regulation of carotenoid biosynthetic process, up-regulation of carotenoid formation, up-regulation of carotenoid synthesis, upregulation of carotenoid anabolism, upregulation of carotenoid biosynthesis, upregulation of carotenoid biosynthetic process, upregulation of carotenoid formation, upregulation of carotenoid synthesis, activation of carotenoid anabolism, activation of carotenoid biosynthesis, activation of carotenoid biosynthetic process, activation of carotenoid formation, activation of carotenoid synthesis Relationships: is a type of regulation of isoprenoid metabolic process [GO:0019747]; is_a GO:0046889; positively regulates carotenoid biosynthetic process [GO:0016117] References: PMID:25675505 Sources: GOC:TermGenie, GO_REF:0000058